male meiotic chromosome movement towards spindle pole [GO:0016346] (biological process) Relationships: is a type of meiotic chromosome movement towards spindle pole [GO:0016344]; is part of male meiosis chromosome segregation [GO:0007060] Also known as: male meiotic chromosome movement, chromosome movement towards spindle pole during male meiosis, male meiotic chromosome movement to spindle pole Definition: The directed movement of chromosomes in the center of the spindle towards the spindle poles, mediated by the shortening of microtubules attached to the chromosomes, during male meiosis. Sources: GOC:ai